histone H2AR3 arginine deiminase activity [GO:0140811] (molecular function) Definition: Catalysis of the reaction: H2O + histone 2A L-arginyl (position 3)= histone 2A L-citrullyl (position 3) + NH4+, resulting in histone H2A citrullination at position 3. References: PMID:15823041 Also known as: H2A-R3 citrullination, histone H2A-R3 arginine deiminase activity, histone-arginine deiminase activity (H2A-R3 specific) Note: Note that the residue position corresponds to the canonical human H2A2A histone (UniProtKB:Q6FI13); this residue seems to be only present in animals. Residue 1 is the first residue following removal of the initiating Methionine (Met). Note that each histone is encoded by multiple genes, and sequences may vary across different genes within an organism. The substrate for histone deiminase may be methyl-arginine, rather than arginine (see PMID:35197210 and PMID:16567635). Relationships: is_a histone arginine deiminase activity [GO:0140794]